{
  "term_id": "UNKNOWN:0001",
  "gene_symbol": "PLEKHO1",
  "gene_name": "Pleckstrin homology domain-containing family O member 1",
  "gene": "UniProtKB:Q53GL0",
  "term_label": "Unknown molecular function"
}